organic acid binding [GO:0043177] (molecular function) Sources: GOC:jl, ISBN:0198506732 Subtypes: carboxylic acid binding [GO:0031406], alkanesulfonate binding [GO:0043210], suramin binding [GO:0043924] Definition: Binding to an organic acid, any acidic compound containing carbon in covalent linkage. Relationships: is a type of GO:0036094